{
  "term_id": "GO:1901379",
  "term_label": "regulation of potassium ion transmembrane transport",
  "gene": "UniProtKB:Q6PIL6",
  "gene_name": "Kv channel-interacting protein 4",
  "gene_symbol": "KCNIP4"
}